{
  "term_id": "GO:0030154",
  "gene_symbol": "BMPR1B",
  "gene_name": "Bone morphogenetic protein receptor type-1B",
  "gene": "UniProtKB:O00238",
  "term_label": "cell differentiation"
}